{
  "gene_symbol": "KPNA4",
  "gene": "UniProtKB:O00629",
  "gene_name": "Importin subunit alpha-3",
  "term_label": "NLS-bearing protein import into nucleus",
  "term_id": "GO:0006607"
}